{
  "gene": "UniProtKB:Q96G74",
  "gene_symbol": "OTUD5",
  "term_id": "GO:0090090",
  "gene_name": "OTU domain-containing protein 5",
  "term_label": "negative regulation of canonical Wnt signaling pathway"
}